immune response-regulating cell surface receptor signaling pathway involved in phagocytosis [GO:0002433] (biological process) Sources: GOC:add, GOC:bf, GO_REF:0000022, ISBN:0781735149 Subtypes: GO:0038096 Definition: An immune response-regulating cell surface receptor signaling pathway that contributes to the endocytic engulfment of external particulate material by phagocytes. Also known as: immune response-regulating cell surface receptor signalling pathway involved in phagocytosis, phagocytosis triggered by activation of immune response cell surface activating receptor Relationships: is a type of GO:0002252; is a type of immune response-regulating cell surface receptor signaling pathway [GO:0002768]; is part of phagocytosis [GO:0006909]